{
  "term_label": "serine-type endopeptidase activity",
  "term_id": "GO:0004252",
  "gene": "UniProtKB:Q6PEW0",
  "gene_symbol": "PRSS54",
  "gene_name": "Inactive serine protease 54"
}